{
  "gene_symbol": "CCL17",
  "gene": "UniProtKB:Q92583",
  "term_label": "Unknown molecular function",
  "gene_name": "C-C motif chemokine 17",
  "term_id": "UNKNOWN:0001"
}